negative regulation of cytoskeleton organization [GO:0051494] (biological process) Also known as: down regulation of cytoskeleton organization, down-regulation of cytoskeleton organization, downregulation of cytoskeleton organization, negative regulation of cytoskeleton organisation, inhibition of cytoskeleton organization, negative regulation of cytoskeleton organization and biogenesis Definition: Any process that stops, prevents, or reduces the frequency, rate or extent of the formation, arrangement of constituent parts, or disassembly of cytoskeletal structures. Subtypes: GO:0030835, negative regulation of actin filament polymerization [GO:0030837], negative regulation of intermediate filament polymerization [GO:0030840], negative regulation of intermediate filament depolymerization [GO:0030843], negative regulation of microtubule polymerization or depolymerization [GO:0031111], negative regulation of actin filament bundle assembly [GO:0032232], negative regulation of centrosome cycle [GO:0046606], negative regulation of actin nucleation [GO:0051126], negative regulation of sarcomere organization [GO:0060299], negative regulation of pseudohyphal septin ring assembly [GO:0062166], negative regulation of mitotic spindle elongation (spindle phase three) [GO:0110163], negative regulation of actin cortical patch assembly [GO:0120133], negative regulation of myosin II filament organization [GO:1904900], negative regulation of cardiac myofibril assembly [GO:1905305], negative regulation of spindle assembly [GO:1905831], negative regulation of cytokinesis, actomyosin contractile ring assembly [GO:2000432] Sources: GOC:ai Relationships: is_a GO:0010639; is a type of regulation of cytoskeleton organization [GO:0051493]; negatively regulates GO:0007010